fusion cell fate specification [GO:0035156] (biological process) Definition: The process in which a cell becomes capable of differentiating autonomously into a fusion cell in an environment that is neutral with respect to the developmental pathway; upon specification, the cell fate can be reversed. Fusion cells allow the interconnection of adjacent tracheal metameres during tracheal tube fusion. Relationships: is_a epithelial cell type specification, open tracheal system [GO:0035153] Regulation: RO_0002212 by negative regulation of fusion cell fate specification [GO:0035157] References: PMID:11063940